{
  "gene_symbol": "MST1R",
  "gene": "UniProtKB:Q04912",
  "term_label": "phagocytosis",
  "term_id": "GO:0006909",
  "gene_name": "Macrophage-stimulating protein receptor"
}